{
  "gene": "UniProtKB:A0A8V8TPW1",
  "gene_name": "Uncharacterized protein",
  "term_label": "Unknown cellular component",
  "term_id": "UNKNOWN:0003",
  "gene_symbol": "A0A8V8TPW1"
}